{
  "gene_name": "Lysosome-associated membrane glycoprotein 2",
  "term_label": "autophagosome maturation",
  "gene": "UniProtKB:P13473",
  "term_id": "GO:0097352",
  "gene_symbol": "LAMP2"
}